{
  "term_id": "UNKNOWN:0001",
  "gene": "UniProtKB:Q8WYR4",
  "gene_name": "Radial spoke head 1 homolog",
  "term_label": "Unknown molecular function",
  "gene_symbol": "RSPH1"
}